peptidyl-serine acetylation [GO:0030920] (biological process) Subtypes: peptidyl-serine O-acetylation [GO:0030919] Relationships: is a type of protein acetylation [GO:0006473] Sources: GOC:mah Definition: The acetylation of peptidyl-serine.